{
  "gene_name": "Caveolae-associated protein 1",
  "term_id": "GO:0005901",
  "term_label": "caveola",
  "gene_symbol": "CAVIN1",
  "gene": "UniProtKB:Q6NZI2"
}